{
  "term_label": "regulation of mRNA stability",
  "gene": "UniProtKB:P51114",
  "gene_name": "RNA-binding protein FXR1",
  "term_id": "GO:0043488",
  "gene_symbol": "FXR1"
}